{
  "gene_symbol": "C1orf159",
  "gene_name": "Uncharacterized protein C1orf159",
  "gene": "UniProtKB:Q96HA4",
  "term_label": "Unknown cellular component",
  "term_id": "UNKNOWN:0003"
}